{
  "gene": "UniProtKB:P09919",
  "gene_name": "Granulocyte colony-stimulating factor",
  "gene_symbol": "CSF3",
  "term_id": "GO:0038158",
  "term_label": "granulocyte colony-stimulating factor signaling pathway"
}